{
  "term_id": "GO:0005883",
  "term_label": "neurofilament",
  "gene": "UniProtKB:P12036",
  "gene_symbol": "NEFH",
  "gene_name": "Neurofilament heavy polypeptide"
}